{
  "term_id": "UNKNOWN:0001",
  "gene_name": "Protein adenylyltransferase SelO, mitochondrial",
  "term_label": "Unknown molecular function",
  "gene_symbol": "SELENOO",
  "gene": "UniProtKB:Q9BVL4"
}